{
  "gene": "UniProtKB:P23219",
  "gene_name": "Prostaglandin G_H synthase 1",
  "gene_symbol": "PTGS1",
  "term_label": "cyclooxygenase pathway",
  "term_id": "GO:0019371"
}